vitamin D response element binding [GO:0070644] (molecular function) Definition: Binding to a vitamin D response element (VDRE), a short sequence with dyad symmetry found in the promoters of some of the cellular immediate-early genes, regulated by serum. Also known as: VDRE binding Relationships: is a type of RNA polymerase II cis-regulatory region sequence-specific DNA binding [GO:0000978] References: PMID:17426122 Sources: GOC:BHF, GOC:vk